{
  "gene_symbol": "PFN1",
  "term_id": "GO:0032233",
  "gene": "UniProtKB:P07737",
  "gene_name": "Profilin-1",
  "term_label": "positive regulation of actin filament bundle assembly"
}